intestinal epithelial cell development [GO:0060576] (biological process) Regulation: RO_0002211 by regulation of intestinal epithelial cell development [GO:1905298]; negatively regulated by negative regulation of intestinal epithelial cell development [GO:1905299]; positively regulated by positive regulation of intestinal epithelial cell development [GO:1905300] Sources: GOC:dph Definition: The process whose specific outcome is the progression of a columnar/cuboidal epithelial cell of the intestine over time, from its formation to the mature structure. Relationships: is a type of columnar/cuboidal epithelial cell development [GO:0002066]; is part of intestinal epithelial cell differentiation [GO:0060575]